{
  "term_label": "extracellular matrix structural constituent",
  "gene_symbol": "NTN5",
  "term_id": "GO:0005201",
  "gene_name": "Netrin-5",
  "gene": "UniProtKB:Q8WTR8"
}